dammarenediol 12-hydroxylase activity [GO:0102556] (molecular function) Relationships: is a type of oxidoreductase activity, acting on paired donors, with incorporation or reduction of molecular oxygen, NAD(P)H as one donor, and incorporation of one atom of oxygen [GO:0016709] Sources: EC:1.14.14.120, GOC:pz Definition: Catalysis of the reaction: dammarenediol-II + NADPH + H+ + O2 = (20S)-protopanaxadiol + NADP + H2O.